{
  "gene_symbol": "ZNF75D",
  "gene": "UniProtKB:P51815",
  "gene_name": "Zinc finger protein 75D",
  "term_label": "RNA polymerase II cis-regulatory region sequence-specific DNA binding",
  "term_id": "GO:0000978"
}